{
  "gene_symbol": "GPHN",
  "term_label": "cytosol",
  "gene_name": "Gephyrin",
  "gene": "UniProtKB:Q9NQX3",
  "term_id": "GO:0005829"
}